{
  "term_label": "DNA binding",
  "term_id": "GO:0003677",
  "gene": "UniProtKB:O60281",
  "gene_name": "Zinc finger protein 292",
  "gene_symbol": "ZNF292"
}